C4-dicarboxylate transmembrane transporter activity [GO:0015556] (molecular function) Sources: GOC:krc Relationships: is a type of carboxylic acid transmembrane transporter activity [GO:0046943]; BFO_0000050 GO:0015740 Definition: Enables the transfer of C4-dicarboxylate from one side of a membrane to the other. Subtypes: oxaloacetate transmembrane transporter activity [GO:0015131], fumarate transmembrane transporter activity [GO:0015138], GO:0015140, succinate transmembrane transporter activity [GO:0015141], GO:0015183, aspartate:alanine antiporter activity [GO:0070906], D-aspartate transmembrane transporter activity [GO:0140010]